{
  "gene_symbol": "KRT7",
  "gene": "UniProtKB:P08729",
  "gene_name": "Keratin, type II cytoskeletal 7",
  "term_id": "GO:0045095",
  "term_label": "keratin filament"
}